{
  "gene": "UniProtKB:Q8IYD9",
  "gene_name": "Lung adenoma susceptibility protein 2",
  "term_id": "UNKNOWN:0002",
  "term_label": "Unknown biological process",
  "gene_symbol": "LAS2"
}